ERBB3-ERBB4 signaling pathway [GO:0038136] (biological process) Definition: The series of molecular signals transmitted by a heterodimeric complex of the tyrosine kinase receptors ERBB3 and ERBB4. The pathway begins with binding of a ligand to either cell surface receptor, or the dimeric receptor complex, and ends with regulation of a downstream cellular process, e.g. transcription. References: PMID:16460914 Sources: GOC:signaling Also known as: ERBB3-ERBB4 signalling pathway, HER3-HER4 signaling pathway Relationships: is a type of ERBB3 signaling pathway [GO:0038129]; is_a ERBB4 signaling pathway [GO:0038130]